{
  "gene_name": "Sodium_nucleoside cotransporter 1",
  "term_id": "GO:0015861",
  "gene_symbol": "SLC28A1",
  "gene": "UniProtKB:O00337",
  "term_label": "cytidine transport"
}